{
  "gene": "UniProtKB:Q8IV53",
  "term_label": "endocytosis",
  "gene_name": "DENN domain-containing protein 1C",
  "term_id": "GO:0006897",
  "gene_symbol": "DENND1C"
}